macrophage migration inhibitory factor receptor complex [GO:0035692] (cellular component) Definition: A protein complex that binds macrophage migration inhibitory factor. Comprises CD74 and CD44 cell surface proteins. Relationships: is a type of receptor complex [GO:0043235] References: PMID:12782713, PMID:17045821 Sources: GOC:BHF